TORC1 complex assembly [GO:1905669] (biological process) Also known as: TOR complex 1 assembly, TOR complex 1 formation, TORC 1 complex assembly, TORC 1 complex formation, TORC1 assembly, TORC1 complex formation, TORC1 formation, nutrient sensitive complex assembly, nutrient sensitive complex formation, rapamycin and nutrient-sensitive TOR complex assembly, rapamycin and nutrient-sensitive TOR complex formation, dTOR/dRaptor complex assembly, dTOR/dRaptor complex formation, dTORC1 assembly, dTORC1 formation, mTORC1 assembly, mTORC1 formation References: PMID:21952218 Sources: GOC:TermGenie, GOC:kmv, GO_REF:0000079 Definition: The aggregation, arrangement and bonding together of a set of components to form a TORC1 complex. Relationships: is a type of protein-containing complex assembly [GO:0065003]